{
  "term_label": "endoplasmic reticulum to Golgi vesicle-mediated transport",
  "gene_name": "Protein transport protein Sec16B",
  "gene": "UniProtKB:Q96JE7",
  "term_id": "GO:0006888",
  "gene_symbol": "SEC16B"
}